{
  "term_id": "UNKNOWN:0002",
  "gene_name": "Putative uncharacterized protein UNQ5815_PRO19632",
  "gene_symbol": "UNQ5815_PRO19632",
  "gene": "UniProtKB:Q6UWF5",
  "term_label": "Unknown biological process"
}